positive regulation of fatty acid transport [GO:2000193] (biological process) Relationships: is a type of positive regulation of lipid transport [GO:0032370]; is a type of positive regulation of organic acid transport [GO:0032892]; is_a regulation of fatty acid transport [GO:2000191]; positively regulates fatty acid transport [GO:0015908] Subtypes: GO:0032305, positive regulation of long-chain fatty acid import into cell [GO:0140214] Definition: Any process that activates or increases the frequency, rate or extent of fatty acid transport. Sources: GOC:BHF